{
  "gene_name": "Serine--tRNA ligase, mitochondrial",
  "term_label": "mitochondrial seryl-tRNA aminoacylation",
  "term_id": "GO:0070158",
  "gene_symbol": "SARS2",
  "gene": "UniProtKB:Q9NP81"
}